{
  "term_id": "UNKNOWN:0001",
  "gene_symbol": "TMED5",
  "term_label": "Unknown molecular function",
  "gene_name": "Transmembrane emp24 domain-containing protein 5",
  "gene": "UniProtKB:Q9Y3A6"
}